{
  "term_label": "microtubule plus-end",
  "gene": "UniProtKB:Q96DZ5",
  "term_id": "GO:0035371",
  "gene_name": "CAP-Gly domain-containing linker protein 3",
  "gene_symbol": "CLIP3"
}